maintenance of protein location in mast cell secretory granule [GO:0033370] (biological process) Subtypes: maintenance of protease location in mast cell secretory granule [GO:0033373] Definition: A process in which a protein is maintained in a secretory granule in a mast cell and prevented from moving elsewhere. Sources: GOC:dph, GOC:mah, GOC:tb Also known as: mast cell protein retention, maintenance of protein localization in mast cell secretory granule Relationships: is a type of maintenance of protein location in cell [GO:0032507]; BFO_0000050 protein localization to mast cell secretory granule [GO:0033367]